{
  "gene_symbol": "TLE1",
  "term_id": "GO:0003714",
  "gene": "UniProtKB:Q04724",
  "gene_name": "Transducin-like enhancer protein 1",
  "term_label": "transcription corepressor activity"
}